{
  "term_id": "GO:0009986",
  "gene": "UniProtKB:O60896",
  "gene_name": "Receptor activity-modifying protein 3",
  "term_label": "cell surface",
  "gene_symbol": "RAMP3"
}